{
  "term_id": "GO:0004771",
  "gene_name": "Bile salt-activated lipase",
  "term_label": "sterol ester esterase activity",
  "gene_symbol": "CEL",
  "gene": "UniProtKB:P19835"
}